{
  "gene": "UniProtKB:O95843",
  "gene_symbol": "GUCA1C",
  "gene_name": "Guanylyl cyclase-activating protein 3",
  "term_id": "UNKNOWN:0003",
  "term_label": "Unknown cellular component"
}